regulation of mitotic telomere tethering at nuclear periphery [GO:1904536] (biological process) Definition: Any process that modulates the frequency, rate or extent of mitotic telomere tethering at nuclear periphery. References: PMID:22959349 Sources: GOC:TermGenie, GO_REF:0000058 Relationships: is a type of GO:0032879; regulates mitotic telomere tethering at nuclear periphery [GO:0044820] Subtypes: negative regulation of mitotic telomere tethering at nuclear periphery [GO:1904537]